mast cell cytokine production [GO:0032762] (biological process) Regulation: regulated by regulation of mast cell cytokine production [GO:0032763]; negatively regulated by negative regulation of mast cell cytokine production [GO:0032764]; positively regulated by positive regulation of mast cell cytokine production [GO:0032765] Note: Note that this term is in the subset of terms that should not be used for direct gene product annotation. Instead, select one of the 'regulation' children terms. Relationships: is a type of myeloid leukocyte cytokine production [GO:0061082] Definition: Any process that contributes to cytokine production by a mast cell. Sources: GOC:mah